potassium channel inhibitor activity [GO:0019870] (MF) Subtypes: inward rectifier potassium channel inhibitor activity [GO:0070320], GO:0140628, small conductance calcium-activated potassium channel inhibitor activity [GO:0140629] Relationships: is a type of GO:0008200; is a type of potassium channel regulator activity [GO:0015459]; negatively regulates potassium channel activity [GO:0005267] Definition: Binds to and stops, prevents, or reduces the activity of a potassium channel. Sources: GOC:mah